{
  "term_label": "Unknown biological process",
  "gene_symbol": "OR52E1",
  "gene": "UniProtKB:Q8NGJ3",
  "gene_name": "Olfactory receptor 52E1",
  "term_id": "UNKNOWN:0002"
}